3-deoxy-manno-octulosonate cytidylyltransferase activity [GO:0008690] (molecular function) Sources: EC:2.7.7.38 Relationships: is a type of GO:0070567 Definition: Catalysis of the reaction: CTP + 3-deoxy-D-manno-octulosonate = diphosphate + CMP-3-deoxy-D-manno-octulosonate. Also known as: CTP:3-deoxy-manno-octulosonate cytidylyltransferase activity, 2-keto-3-deoxyoctonate cytidylyltransferase activity, 3-deoxy-D-manno-octulosonate cytidylyltransferase activity, CMP-2-keto-3-deoxyoctulosonic acid synthetase activity, CMP-3-deoxy-D-manno-octulosonate diphosphorylase activity, CMP-3-deoxy-D-manno-octulosonate pyrophosphorylase activity, CMP-3-deoxy-D-manno-octulosonate synthetase activity, CMP-KDO synthetase activity, CTP:3-deoxy-D-manno-octulosonate cytidylyltransferase activity, CTP:CMP-3-deoxy-D-manno-octulosonate cytidylyltransferase activity, cytidine monophospho-3-deoxy-D-manno-octulosonate pyrophosphorylase activity